{
  "gene_symbol": "TFAP2E",
  "gene_name": "Transcription factor AP-2-epsilon",
  "term_label": "nucleus",
  "term_id": "GO:0005634",
  "gene": "UniProtKB:Q6VUC0"
}